{
  "term_id": "UNKNOWN:0003",
  "gene_name": "SLIT-ROBO Rho GTPase-activating protein 1",
  "gene": "UniProtKB:Q7Z6B7",
  "gene_symbol": "SRGAP1",
  "term_label": "Unknown cellular component"
}